{
  "gene_symbol": "LGI3",
  "gene_name": "Leucine-rich repeat LGI family member 3",
  "term_label": "Unknown molecular function",
  "gene": "UniProtKB:Q8N145",
  "term_id": "UNKNOWN:0001"
}